daunorubicin biosynthetic process [GO:1901771] (biological process) References: PMID:7601857 Sources: GOC:TermGenie, GOC:yaf, UniPathway:UPA00054 Definition: The chemical reactions and pathways resulting in the formation of daunorubicin. Also known as: daunorubicin anabolism, daunorubicin biosynthesis, daunorubicin formation, daunorubicin synthesis Relationships: is a type of polyketide biosynthetic process [GO:0030639]; is a type of GO:0030648; is_a ketone biosynthetic process [GO:0042181]; is a type of daunorubicin metabolic process [GO:0044597]